narrow pore, gated channel activity [GO:0022831] (molecular function) Sources: GOC:mtg_transport, ISBN:0815340729 Relationships: is a type of narrow pore channel activity [GO:0022842] Also known as: ion channels Definition: Enables the transport of a solute across a membrane via a narrow pore channel that opens in response to a particular stimulus.